{
  "term_id": "GO:0007165",
  "gene_name": "Protein FAM3B",
  "gene_symbol": "FAM3B",
  "term_label": "signal transduction",
  "gene": "UniProtKB:P58499"
}